{
  "term_label": "cytosol",
  "gene": "UniProtKB:Q9H008",
  "gene_symbol": "LHPP",
  "gene_name": "Phospholysine phosphohistidine inorganic pyrophosphate phosphatase",
  "term_id": "GO:0005829"
}